{
  "gene_symbol": "IGHG2",
  "gene_name": "Immunoglobulin heavy constant gamma 2",
  "term_id": "GO:0006958",
  "gene": "UniProtKB:P01859",
  "term_label": "complement activation, classical pathway"
}